cytosolic proteasome core complex, beta-subunit complex [GO:0031609] (cellular component) Sources: GOC:mah, GOC:mtg_sensu Definition: The proteasome core subcomplex that constitutes the two inner rings of the cytosolic proteasome core complex. Relationships: is a type of proteasome core complex, beta-subunit complex [GO:0019774]; is part of cytosolic proteasome core complex [GO:0031603]